positive regulation of chemotaxis to cAMP by DIF-2 [GO:0061128] (biological process) Sources: GOC:dph Definition: Any process that increases the rate, frequency, or extent of directed movement of a motile cell or organism up a concentration gradient of 3',5'-cAMP by the action of DIF-2. DIF-2 is a chlorinated alkylphenone. Relationships: is a type of regulation of positive chemotaxis to cAMP by DIF-2 [GO:0061121]; is a type of positive regulation of positive chemotaxis to cAMP by chlorinated alkylphenone [GO:0061124]